{
  "term_id": "GO:0097192",
  "gene_symbol": "BCL2",
  "term_label": "extrinsic apoptotic signaling pathway in absence of ligand",
  "gene_name": "Apoptosis regulator Bcl-2",
  "gene": "UniProtKB:P10415"
}